{
  "gene": "UniProtKB:Q9H3S1",
  "gene_name": "Semaphorin-4A",
  "gene_symbol": "SEMA4A",
  "term_label": "chemorepellent activity",
  "term_id": "GO:0045499"
}